{
  "gene_symbol": "TRIM5",
  "gene": "UniProtKB:Q9C035",
  "term_id": "GO:0032880",
  "term_label": "regulation of protein localization",
  "gene_name": "Tripartite motif-containing protein 5"
}